{
  "gene_name": "General transcription factor 3C polypeptide 5",
  "gene_symbol": "GTF3C5",
  "term_id": "GO:0042791",
  "gene": "UniProtKB:Q9Y5Q8",
  "term_label": "5S class rRNA transcription by RNA polymerase III"
}